{
  "gene_symbol": "ADRB1",
  "term_label": "positive regulation of MAPK cascade",
  "gene": "UniProtKB:P08588",
  "gene_name": "Beta-1 adrenergic receptor",
  "term_id": "GO:0043410"
}